{
  "gene": "UniProtKB:O14791",
  "term_id": "UNKNOWN:0002",
  "gene_symbol": "APOL1",
  "term_label": "Unknown biological process",
  "gene_name": "Apolipoprotein L1"
}